putrescine N-methyltransferase activity [GO:0030750] (molecular function) Relationships: is a type of GO:0008757 Also known as: S-adenosyl-L-methionine:putrescine N-methyltransferase activity, putrescine methyltransferase activity Definition: Catalysis of the reaction: S-adenosyl-L-methionine + putrescine = N-methylputrescine + S-adenosyl-L-homocysteine + H+. Sources: EC:2.1.1.53, RHEA:15037